negative regulation of vascular endothelial growth factor signaling pathway [GO:1900747] (biological process) Definition: Any process that stops, prevents or reduces the frequency, rate or extent of vascular endothelial growth factor signaling pathway. Also known as: down regulation of VEGF signaling, down regulation of VEGF-activated signaling pathway, down regulation of vascular endothelial growth factor signaling pathway, down regulation of vascular endothelial growth factor signalling pathway, down-regulation of VEGF signaling, down-regulation of VEGF-activated signaling pathway, down-regulation of vascular endothelial growth factor signaling pathway, down-regulation of vascular endothelial growth factor signalling pathway, downregulation of VEGF signaling, downregulation of VEGF-activated signaling pathway, downregulation of vascular endothelial growth factor signaling pathway, downregulation of vascular endothelial growth factor signalling pathway, inhibition of VEGF signaling, inhibition of VEGF-activated signaling pathway, inhibition of vascular endothelial growth factor signalling pathway, negative regulation of VEGF signaling, negative regulation of VEGF-activated signaling pathway, negative regulation of vascular endothelial growth factor signalling pathway, inhibition of vascular endothelial growth factor signaling pathway Sources: GOC:TermGenie Relationships: is a type of GO:0009968; is a type of regulation of vascular endothelial growth factor signaling pathway [GO:1900746]; is_a negative regulation of cellular response to vascular endothelial growth factor stimulus [GO:1902548]; negatively regulates vascular endothelial growth factor signaling pathway [GO:0038084]